{
  "gene_name": "Creatine kinase S-type, mitochondrial",
  "gene": "UniProtKB:P17540",
  "term_label": "creatine kinase activity",
  "term_id": "GO:0004111",
  "gene_symbol": "CKMT2"
}